positive regulation of interleukin-1 beta production [GO:0032731] (biological process) Sources: GOC:mah Relationships: is a type of regulation of interleukin-1 beta production [GO:0032651]; is a type of positive regulation of interleukin-1 production [GO:0032732]; positively regulates interleukin-1 beta production [GO:0032611] Definition: Any process that activates or increases the frequency, rate, or extent of interleukin-1 beta production. Also known as: positive regulation of IL-1 beta production, up regulation of interleukin-1 beta production, up-regulation of interleukin-1 beta production, upregulation of interleukin-1 beta production, activation of interleukin-1 beta production, positive regulation of interleukin-1 beta biosynthetic process, positive regulation of interleukin-1 beta secretion, stimulation of interleukin-1 beta production